invasive growth in response to biotic stimulus [GO:0097317] (biological process) Definition: The growth of colonies in filamentous chains of cells as a result of a biotic stimulus. An example of this is Candida albicans forming invasive filaments in agar medium in response to a serum stimulus. References: PMID:18679170 Sources: GOC:di Relationships: is a type of filamentous growth of a population of unicellular organisms in response to biotic stimulus [GO:0036180]; is a type of invasive filamentous growth [GO:0036267]